regulation of neuroblast proliferation [GO:1902692] (biological process) Definition: Any process that modulates the frequency, rate or extent of neuroblast proliferation. Subtypes: positive regulation of neuroblast proliferation [GO:0002052], negative regulation of neuroblast proliferation [GO:0007406] Relationships: is a type of regulation of neural precursor cell proliferation [GO:2000177]; regulates neuroblast proliferation [GO:0007405] References: PMID:21168496 Sources: GOC:PARL, GOC:TermGenie, GOC:rl, GO_REF:0000058